{
  "gene_symbol": "TCF12",
  "term_id": "GO:0000981",
  "gene_name": "Transcription factor 12",
  "gene": "UniProtKB:Q99081",
  "term_label": "DNA-binding transcription factor activity, RNA polymerase II-specific"
}